{
  "gene": "UniProtKB:Q5VZ52",
  "gene_symbol": "MORN5",
  "term_id": "UNKNOWN:0003",
  "gene_name": "MORN repeat-containing protein 5",
  "term_label": "Unknown cellular component"
}